1,3-beta-galactosyl-N-acetylhexosamine phosphorylase activity [GO:0050500] (molecular function) Relationships: is a type of hexosyltransferase activity [GO:0016758] Definition: Catalysis of the reaction: phosphate + beta-D-galactopyranosyl-(1->3)-N-acetyl-D-glucosamine = N-acetyl-D-glucosamine + alpha-D-galactopyranose 1-phosphate. Also known as: beta-1,3-galactosyl-N-acetylhexosamine phosphorylase activity, beta-D-galactopyranosyl-(1,3)-N-acetyl-D-hexosamine:phosphate galactosyltransferase activity, beta-D-galactopyranosyl-(1->3)-N-acetyl-D-hexosamine:phosphate galactosyltransferase activity Sources: EC:2.4.1.211, MetaCyc:2.4.1.211-RXN